cardiac left atrium morphogenesis [GO:0003212] (biological process) Definition: The process in which the left cardiac atrium is generated and organized. Sources: GOC:mtg_heart Relationships: is a type of cardiac atrium morphogenesis [GO:0003209]